{
  "gene_name": "Myotubularin",
  "term_id": "GO:0048311",
  "term_label": "mitochondrion distribution",
  "gene": "UniProtKB:Q13496",
  "gene_symbol": "MTM1"
}